{
  "gene_symbol": "EBF4",
  "term_id": "GO:0000981",
  "gene_name": "Transcription factor COE4",
  "gene": "UniProtKB:Q9BQW3",
  "term_label": "DNA-binding transcription factor activity, RNA polymerase II-specific"
}